{
  "gene_symbol": "ITGB3",
  "term_label": "cell-matrix adhesion",
  "term_id": "GO:0007160",
  "gene": "UniProtKB:P05106",
  "gene_name": "Integrin beta-3"
}